{
  "gene_name": "ATP synthase subunit epsilon-like protein, mitochondrial",
  "gene": "UniProtKB:Q5VTU8",
  "term_id": "GO:0005743",
  "term_label": "mitochondrial inner membrane",
  "gene_symbol": "ATP5F1EP2"
}